detoxification of aluminum ion [GO:0140982] (biological process) Relationships: is a type of detoxification of inorganic compound [GO:0061687] Definition: Any process that reduce or remove the toxicity of aluminum ions. These can include transport of the aluminum away from sensitive areas, sequesteration, or chemical modification to an inert form. References: PMID:10845450, PMID:23888867, PMID:9576769 Also known as: aluminum ion homeostasis